{
  "term_label": "synaptic membrane",
  "gene_symbol": "AKAP9",
  "term_id": "GO:0097060",
  "gene": "UniProtKB:Q99996",
  "gene_name": "A-kinase anchor protein 9"
}